nicotinate phosphoribosyltransferase activity [GO:0004516] (molecular function) Definition: Catalysis of the reaction: nicotinate + 5-phospho-alpha-D-ribose 1-diphosphate + ATP + H2O = nicotinate beta-D-ribonucleotide + ADP + phosphate + diphosphate. Relationships: is a type of ligase activity, forming carbon-nitrogen bonds [GO:0016879] References: PMID:7503993 Sources: RHEA:36163 Also known as: niacin ribonucleotidase activity, nicotinate-nucleotide:diphosphate phospho-alpha-D-ribosyltransferase activity, nicotinic acid mononucleotide glycohydrolase activity, nicotinic acid mononucleotide pyrophosphorylase activity, nicotinic acid phosphoribosyltransferase activity